{
  "gene_name": "Single-stranded DNA-binding protein 3",
  "gene_symbol": "SSBP3",
  "term_id": "GO:0003713",
  "gene": "UniProtKB:Q9BWW4",
  "term_label": "transcription coactivator activity"
}